{
  "term_label": "SNARE binding",
  "gene_name": "Synaptotagmin-4",
  "gene_symbol": "SYT4",
  "term_id": "GO:0000149",
  "gene": "UniProtKB:Q9H2B2"
}